{
  "term_id": "UNKNOWN:0003",
  "gene_name": "Max dimerization protein 4",
  "term_label": "Unknown cellular component",
  "gene_symbol": "MXD4",
  "gene": "UniProtKB:Q14582"
}